{
  "gene_symbol": "IP6K3",
  "gene": "UniProtKB:Q96PC2",
  "term_id": "GO:0046854",
  "gene_name": "Inositol hexakisphosphate kinase 3",
  "term_label": "phosphatidylinositol phosphate biosynthetic process"
}